{
  "gene_name": "Arrestin domain-containing protein 5",
  "gene_symbol": "ARRDC5",
  "term_id": "GO:0005768",
  "term_label": "endosome",
  "gene": "UniProtKB:A6NEK1"
}